{
  "gene_name": "Transmembrane 6 superfamily member 2",
  "term_id": "GO:0055088",
  "gene": "UniProtKB:Q9BZW4",
  "term_label": "lipid homeostasis",
  "gene_symbol": "TM6SF2"
}